{
  "gene_symbol": "GUCY2F",
  "gene": "UniProtKB:P51841",
  "term_label": "plasma membrane",
  "gene_name": "Retinal guanylyl cyclase 2",
  "term_id": "GO:0005886"
}